JUN kinase activity [GO:0004705] (molecular function) Definition: Catalysis of the reaction: JUN + ATP = JUN phosphate + ADP. This reaction is the phosphorylation and activation of members of the JUN family, a gene family that encodes nuclear transcription factors. Regulation: regulated by regulation of JUN kinase activity [GO:0043506]; positively regulated by positive regulation of JUN kinase activity [GO:0043507]; negatively regulated by GO:0043508 Also known as: JNK, SAPK1, c-Jun N-terminal kinase activity, JNK3alpha1 Sources: GOC:bf, ISBN:0198506732 Relationships: is a type of MAP kinase activity [GO:0004707]; is part of JNK cascade [GO:0007254]